{
  "gene": "UniProtKB:P21817",
  "term_id": "GO:0005790",
  "term_label": "smooth endoplasmic reticulum",
  "gene_symbol": "RYR1",
  "gene_name": "Ryanodine receptor 1"
}